{
  "gene_name": "Double homeobox protein 4-like protein 7",
  "gene_symbol": "DUX4L7",
  "term_label": "RNA polymerase II transcription regulatory region sequence-specific DNA binding",
  "gene": "UniProtKB:P0CJ90",
  "term_id": "GO:0000977"
}